positive regulation of strand invasion [GO:0098530] (biological process) Also known as: positive regulation of Rad51-mediated strand invasion, positive regulation of D-loop biosynthesis, positive regulation of D-loop formation Sources: GOC:dos, GOC:dph, GOC:elh, GOC:tb Relationships: is a type of positive regulation of DNA metabolic process [GO:0051054]; is a type of regulation of strand invasion [GO:0060542]; positively regulates GO:0042148 Definition: Any process that increases the rate, frequency or extent of strand invasion. Strand invasion is the process in which the nucleoprotein complex (composed of the broken single-strand DNA and the recombinase) searches and identifies a region of homology in intact duplex DNA. The broken single-strand DNA displaces the like strand and forms Watson-Crick base pairs with its complement, forming a duplex in which each strand is from one of the two recombining DNA molecules.